{
  "gene_name": "Scavenger receptor cysteine-rich domain-containing group B protein",
  "term_id": "GO:0005044",
  "gene": "UniProtKB:Q8WTU2",
  "term_label": "scavenger receptor activity",
  "gene_symbol": "SSC4D"
}